{
  "gene_symbol": "LBP",
  "term_label": "defense response to Gram-positive bacterium",
  "gene": "UniProtKB:P18428",
  "term_id": "GO:0050830",
  "gene_name": "Lipopolysaccharide-binding protein"
}